farnesyl diphosphate biosynthetic process, mevalonate pathway [GO:0010142] (biological process) Sources: GOC:pz, MetaCyc:PWY-922 Definition: The pathway that converts acetate, in the form of acetyl-CoA, to farnesyl diphosphate (FPP) through a series of mevalonate intermediates. Farnesyl diphosphate is an important substrate for other essential pathways, such as biosynthesis of sterols. Also known as: farnesyl diphosphate anabolism, mevalonate pathway, farnesyl diphosphate formation, mevalonate pathway, farnesyl diphosphate synthesis, mevalonate pathway, isoprenoid pathway, Ac-MVA pathway, acetate-mevalonate pathway Relationships: is a type of farnesyl diphosphate biosynthetic process [GO:0045337]; is a type of GO:1902767